{
  "term_label": "mitotic sister chromatid cohesion",
  "gene": "UniProtKB:Q9UQE7",
  "gene_symbol": "SMC3",
  "gene_name": "Structural maintenance of chromosomes protein 3",
  "term_id": "GO:0007064"
}